{
  "gene": "UniProtKB:Q99062",
  "gene_symbol": "CSF3R",
  "term_id": "GO:0004896",
  "gene_name": "Granulocyte colony-stimulating factor receptor",
  "term_label": "cytokine receptor activity"
}